{
  "gene": "UniProtKB:P60981",
  "term_label": "actin filament binding",
  "term_id": "GO:0051015",
  "gene_symbol": "DSTN",
  "gene_name": "Destrin"
}